cellular response to cordycepin [GO:1904310] (biological process) Relationships: is a type of GO:1901699; is a type of cellular response to oxygen-containing compound [GO:1901701]; is a type of response to cordycepin [GO:1904309] Also known as: cellular response to 3'-deoxyadenosine References: PMID:21597460 Sources: GOC:TermGenie, GO_REF:0000071 Definition: Any process that results in a change in state or activity of a cell (in terms of movement, secretion, enzyme production, gene expression, etc.) as a result of a cordycepin stimulus.